quinolinic acid transmembrane transport [GO:1903222] (BP) Definition: The process in which quinolinic acid is transported across a membrane. Relationships: is a type of dicarboxylic acid transport [GO:0006835]; is a type of nitrogen compound transport [GO:0071705]; is_a GO:1905039 References: PMID:23457190 Sources: GOC:TermGenie, GOC:di, GO_REF:0000069